{
  "gene": "UniProtKB:Q9NYW2",
  "gene_name": "Taste receptor type 2 member 8",
  "term_label": "detection of chemical stimulus involved in sensory perception of bitter taste",
  "gene_symbol": "TAS2R8",
  "term_id": "GO:0001580"
}